{
  "gene": "UniProtKB:Q6TGC4",
  "term_label": "cytoplasm",
  "gene_symbol": "PADI6",
  "gene_name": "Protein-arginine deiminase type-6",
  "term_id": "GO:0005737"
}